{
  "gene": "UniProtKB:P20366",
  "gene_symbol": "TAC1",
  "gene_name": "Protachykinin-1",
  "term_id": "GO:0031835",
  "term_label": "substance P receptor binding"
}